regulation of trypanothione biosynthetic process [GO:1905722] (BP) Relationships: is a type of regulation of biosynthetic process [GO:0009889]; is a type of regulation of sulfur metabolic process [GO:0042762]; regulates trypanothione biosynthetic process [GO:0019342] References: PMID:18949025 Sources: GOC:TermGenie, GO_REF:0000058 Definition: Any process that modulates the frequency, rate or extent of trypanothione biosynthetic process. Subtypes: GO:1905723, positive regulation of trypanothione biosynthetic process [GO:1905724] Also known as: regulation of trypanothione anabolism, regulation of trypanothione biosynthesis, regulation of trypanothione formation, regulation of trypanothione synthesis